{
  "term_id": "GO:0070552",
  "gene_symbol": "MPND",
  "gene_name": "MPN domain-containing protein",
  "gene": "UniProtKB:Q8N594",
  "term_label": "BRISC complex"
}